{
  "gene_name": "Spermidine_spermine N(1)-acetyltransferase-like protein 1",
  "gene": "UniProtKB:Q86VE3",
  "term_label": "Unknown cellular component",
  "term_id": "UNKNOWN:0003",
  "gene_symbol": "SATL1"
}